ITP metabolic process [GO:0046041] (biological process) Sources: GOC:go_curators Relationships: is a type of purine ribonucleotide metabolic process [GO:0009150]; is a type of purine ribonucleoside triphosphate metabolic process [GO:0009205] Subtypes: GO:0006193, ITP biosynthetic process [GO:0046042] Definition: The chemical reactions and pathways involving ITP, inosine triphosphate. Also known as: ITP metabolism